{
  "gene_symbol": "INSL5",
  "term_label": "positive regulation of feeding behavior",
  "gene_name": "Insulin-like peptide INSL5",
  "gene": "UniProtKB:Q9Y5Q6",
  "term_id": "GO:2000253"
}